{
  "gene_symbol": "PCMTD1",
  "term_id": "GO:0004719",
  "gene_name": "Protein-L-isoaspartate O-methyltransferase domain-containing protein 1",
  "term_label": "protein-L-isoaspartate (D-aspartate) O-methyltransferase activity",
  "gene": "UniProtKB:Q96MG8"
}